1-methylguanosine metabolic process [GO:0080179] (biological process) Sources: GOC:tb Definition: The chemical reactions and pathways involving 1-methylguanosine. Relationships: is a type of purine ribonucleoside metabolic process [GO:0046128]